mating projection formation [GO:0031382] (biological process) Regulation: regulated by regulation of mating projection assembly [GO:0031383]; positively regulated by positive regulation of mating projection assembly [GO:1902917] Definition: The aggregation, arrangement and bonding together of a set of components to form a cell projection in response to mating pheromone. This process is observed in unicellular fungi. Relationships: is a type of cellular component assembly involved in morphogenesis [GO:0010927]; is a type of plasma membrane bounded cell projection assembly [GO:0120031]; is part of cell morphogenesis involved in conjugation with cellular fusion [GO:0000753] Also known as: mating projection assembly, shmooing, mating projection biogenesis References: PMID:14734532 Sources: GOC:mah